{
  "term_label": "Unknown cellular component",
  "gene_symbol": "SPATA31A5",
  "term_id": "UNKNOWN:0003",
  "gene_name": "Spermatogenesis-associated protein 31A5",
  "gene": "UniProtKB:Q5VU36"
}